{
  "term_label": "rRNA binding",
  "gene_name": "Suppressor of SWI4 1 homolog",
  "term_id": "GO:0019843",
  "gene_symbol": "PPAN",
  "gene": "UniProtKB:Q9NQ55"
}